{
  "gene_name": "Tumor necrosis factor receptor superfamily member EDAR",
  "gene": "UniProtKB:Q9UNE0",
  "gene_symbol": "EDAR",
  "term_label": "positive regulation of canonical NF-kappaB signal transduction",
  "term_id": "GO:0043123"
}